{
  "term_id": "UNKNOWN:0001",
  "term_label": "Unknown molecular function",
  "gene_symbol": "CHERP",
  "gene": "UniProtKB:Q8IWX8",
  "gene_name": "Calcium homeostasis endoplasmic reticulum protein"
}